modification of synaptic structure [GO:0099563] (biological process) Definition: Any process that modifies the structure/morphology of a synapse. Subtypes: modification of postsynaptic structure [GO:0099010], modification of synaptic structure, modulating synaptic transmission [GO:0099564] Sources: GOC:dos Relationships: is a type of synapse organization [GO:0050808] Regulation: regulated by regulation of modification of synaptic structure [GO:1905244] Also known as: synapse remodelling Note: This class does not cover assembly or disassembly of synapses, only the modification/remodelling of existing ones.